{
  "gene": "UniProtKB:Q9H4M7",
  "gene_name": "Pleckstrin homology domain-containing family A member 4",
  "gene_symbol": "PLEKHA4",
  "term_label": "phosphatidylinositol-3,4-bisphosphate binding",
  "term_id": "GO:0043325"
}